{
  "term_label": "perisynaptic extracellular matrix",
  "gene_symbol": "TNC",
  "gene": "UniProtKB:P24821",
  "term_id": "GO:0098966",
  "gene_name": "Tenascin"
}